oleate 12-hydroxylase activity [GO:0102517] (molecular function) Relationships: is_a oxidoreductase activity, acting on paired donors, with incorporation or reduction of molecular oxygen, NAD(P)H as one donor, and incorporation of one atom of oxygen [GO:0016709] Definition: Catalysis of the reaction: (9Z)-octadecenoate + AH2 + O2 = (12R)-hydroxy-(9Z)-octadecenoate + acceptor + H2O. Sources: RHEA:55956